{
  "gene_symbol": "RAB3GAP1",
  "gene_name": "Rab3 GTPase-activating protein catalytic subunit",
  "term_label": "positive regulation of autophagosome assembly",
  "term_id": "GO:2000786",
  "gene": "UniProtKB:Q15042"
}